{
  "term_label": "thyroid hormone metabolic process",
  "gene_symbol": "CRYM",
  "gene": "UniProtKB:Q14894",
  "term_id": "GO:0042403",
  "gene_name": "Ketimine reductase mu-crystallin"
}